{
  "term_label": "RNA polymerase II transcription regulator complex",
  "gene_name": "Transcription intermediary factor 1-beta",
  "gene": "UniProtKB:Q13263",
  "gene_symbol": "TRIM28",
  "term_id": "GO:0090575"
}